{
  "gene_name": "Coatomer subunit gamma-1",
  "term_id": "GO:0000139",
  "gene": "UniProtKB:Q9Y678",
  "gene_symbol": "COPG1",
  "term_label": "Golgi membrane"
}